{
  "gene_symbol": "ENTPD2",
  "term_label": "ribonucleoside triphosphate phosphatase activity",
  "gene_name": "Ectonucleoside triphosphate diphosphohydrolase 2",
  "term_id": "GO:0017111",
  "gene": "UniProtKB:Q9Y5L3"
}